acyl-phosphate glycerol-3-phosphate acyltransferase activity [GO:0043772] (molecular function) Also known as: acyl-phosphate:glycerol-3-phosphate acyltransferase activity, acylphosphate glycerol-3-phosphate acyltransferase activity, acylphosphate:glycerol-3-phosphate acyltransferase activity Definition: Catalysis of the reaction: acyl phosphate + sn-glycerol 3-phosphate = 1-acyl-sn-glycerol 3-phosphate + orthophosphate. Relationships: is a type of acyltransferase activity, transferring groups other than amino-acyl groups [GO:0016747] References: PMID:17308305